{
  "term_label": "nucleotide-activated protein kinase complex",
  "gene_symbol": "PRKAG2",
  "term_id": "GO:0031588",
  "gene": "UniProtKB:Q9UGJ0",
  "gene_name": "5'-AMP-activated protein kinase subunit gamma-2"
}